{
  "term_label": "delta(3)-delta(2)-enoyl-CoA isomerase activity",
  "gene_symbol": "ECI1",
  "gene_name": "Enoyl-CoA delta isomerase 1, mitochondrial",
  "term_id": "GO:0004165",
  "gene": "UniProtKB:P42126"
}